directional locomotion [GO:0033058] (biological process) Sources: GOC:mtg_MIT_16mar07 Subtypes: forward locomotion [GO:0043056], backward locomotion [GO:0043057] Definition: Self-propelled movement of a cell or organism from one location to another along an axis. Relationships: is a type of locomotion [GO:0040011]